{
  "gene_name": "PHD finger protein 24",
  "term_label": "Unknown biological process",
  "gene_symbol": "PHF24",
  "gene": "UniProtKB:Q9UPV7",
  "term_id": "UNKNOWN:0002"
}